{
  "gene_name": "Leucine-rich repeat and fibronectin type-III domain-containing protein 5",
  "term_label": "postsynaptic density membrane",
  "gene_symbol": "LRFN5",
  "term_id": "GO:0098839",
  "gene": "UniProtKB:Q96NI6"
}